{
  "term_id": "GO:0005829",
  "gene": "UniProtKB:P52565",
  "term_label": "cytosol",
  "gene_name": "Rho GDP-dissociation inhibitor 1",
  "gene_symbol": "ARHGDIA"
}